{
  "term_id": "GO:0005637",
  "gene_name": "Delta(14)-sterol reductase TM7SF2",
  "gene": "UniProtKB:O76062",
  "gene_symbol": "TM7SF2",
  "term_label": "nuclear inner membrane"
}